DNA endonuclease activity, producing 5'-phosphomonoesters [GO:0016888] (molecular function) Sources: GOC:ai Relationships: is a type of DNA endonuclease activity [GO:0004520]; is a type of GO:0016788 Also known as: endodeoxyribonuclease activity, producing 5' phosphomonoesters, endodeoxyribonuclease activity, producing 5'-phosphomonoesters Definition: Catalysis of the hydrolysis of ester linkages within deoxyribonucleic acids by creating internal breaks to yield 5'-phosphomonoesters. Subtypes: deoxyribonuclease I activity [GO:0004530], GO:0008833, GO:0009035, GO:0009036, type III site-specific deoxyribonuclease activity [GO:0015668], 5'-flap endonuclease activity [GO:0017108], GO:0033891, deoxyribonuclease V activity [GO:0043737], class II DNA-(apurinic or apyrimidinic site) endonuclease activity [GO:0052720]